{
  "term_id": "GO:0048488",
  "gene": "UniProtKB:O60890",
  "gene_symbol": "OPHN1",
  "term_label": "synaptic vesicle endocytosis",
  "gene_name": "Oligophrenin-1"
}